{
  "gene": "UniProtKB:Q96MZ0",
  "gene_name": "Ganglioside-induced differentiation-associated protein 1-like 1",
  "gene_symbol": "GDAP1L1",
  "term_label": "Unknown molecular function",
  "term_id": "UNKNOWN:0001"
}